symbiont-mediated perturbation of host receptor-mediated signal transduction [GO:0075109] (biological process) Subtypes: symbiont-mediated suppression of host receptor-mediated signal transduction [GO:0075111], GO:0075118, symbiont-mediated suppression of host pro-inflammatory cytokine signaling [GO:0141173], symbiont-mediated suppression of host anti-inflammatory cytokine signaling [GO:0141174] Definition: A process by which a symbiont alters or subverts a receptor-mediated signal transduction pathway in its host organism. The host is defined as the larger of the organisms involved in a symbiotic interaction. Relationships: is a type of symbiont-mediated perturbation of host signal transduction pathway [GO:0052027] Also known as: perturbation of host receptor-mediated signal transduction Sources: GOC:pamgo_curators